dopaminergic synapse [GO:0098691] (cellular component) Relationships: is a type of synapse [GO:0045202] Definition: A synapse that uses dopamine as a neurotransmitter. Sources: GOC:dos